{
  "gene_name": "CD44 antigen",
  "gene": "UniProtKB:P16070",
  "term_label": "inflammatory response",
  "term_id": "GO:0006954",
  "gene_symbol": "CD44"
}